{
  "term_label": "proteolysis",
  "gene_symbol": "ADAM22",
  "term_id": "GO:0006508",
  "gene_name": "Disintegrin and metalloproteinase domain-containing protein 22",
  "gene": "UniProtKB:Q9P0K1"
}